{
  "term_id": "UNKNOWN:0001",
  "term_label": "Unknown molecular function",
  "gene_symbol": "MFSD11",
  "gene": "UniProtKB:O43934",
  "gene_name": "UNC93-like protein MFSD11"
}